{
  "gene": "UniProtKB:P52569",
  "term_id": "GO:1903352",
  "gene_name": "Cationic amino acid transporter 2",
  "term_label": "L-ornithine transmembrane transport",
  "gene_symbol": "SLC7A2"
}